regulation of interleukin-35 production [GO:0070754] (biological process) Also known as: regulation of IL-35 production, regulation of interleukin-35 biosynthetic process Sources: GOC:mah Relationships: is a type of GO:0001817; RO_0002211 interleukin-35 production [GO:0070753] Definition: Any process that modulates the frequency, rate, or extent of interleukin-35 production. Subtypes: GO:0070755, GO:0070756